{
  "gene_name": "Tetra-peptide repeat homeobox-like protein",
  "gene_symbol": "TPRXL",
  "term_id": "UNKNOWN:0002",
  "term_label": "Unknown biological process",
  "gene": "UniProtKB:Q17RH7"
}